chlorophyll synthetase activity [GO:0046408] (molecular function) Relationships: is_a prenyltransferase activity [GO:0004659] Sources: RHEA:17317 Also known as: chlorophyll synthase activity, chlorophyllide-a:phytyl-diphosphate phytyltransferase activity Definition: Catalysis of the reaction: chlorophyllide a + phytyl diphosphate + 2 H+ = chlorophyll a + diphosphate.